{
  "gene": "UniProtKB:Q8NC24",
  "term_id": "UNKNOWN:0001",
  "gene_name": "RELT-like protein 2",
  "term_label": "Unknown molecular function",
  "gene_symbol": "RELL2"
}